{
  "term_label": "Unknown biological process",
  "term_id": "UNKNOWN:0002",
  "gene": "UniProtKB:Q9H342",
  "gene_name": "Olfactory receptor 51J1",
  "gene_symbol": "OR51J1"
}